{
  "gene_name": "Carbonic anhydrase 2",
  "gene_symbol": "CA2",
  "term_label": "carbon dioxide transport",
  "term_id": "GO:0015670",
  "gene": "UniProtKB:P00918"
}